zinc ion import into secretory vesicle [GO:0140914] (biological process) Definition: The directed import of zinc(2+) from the cytosol, across an organelle membrane, into a secretory vesicle. References: PMID:19496757 Relationships: is a type of zinc ion import into organelle [GO:0062111] Subtypes: zinc ion import into zymogen granule [GO:0140915]